{
  "gene_name": "Interferon alpha-4",
  "term_label": "type I interferon receptor binding",
  "gene_symbol": "IFNA4",
  "term_id": "GO:0005132",
  "gene": "UniProtKB:P05014"
}